{
  "gene": "UniProtKB:P49326",
  "term_label": "N,N-dimethylaniline monooxygenase activity",
  "gene_name": "Flavin-containing monooxygenase 5",
  "gene_symbol": "FMO5",
  "term_id": "GO:0004499"
}